{
  "term_id": "GO:0005769",
  "term_label": "early endosome",
  "gene_name": "E3 ubiquitin-protein ligase MGRN1",
  "gene": "UniProtKB:O60291",
  "gene_symbol": "MGRN1"
}